{
  "term_label": "V1A vasopressin receptor binding",
  "gene": "UniProtKB:P01185",
  "gene_symbol": "AVP",
  "gene_name": "Vasopressin-neurophysin 2-copeptin",
  "term_id": "GO:0031894"
}